{
  "term_id": "UNKNOWN:0001",
  "term_label": "Unknown molecular function",
  "gene": "UniProtKB:Q86UP8",
  "gene_name": "General transcription factor II-I repeat domain-containing protein 2A",
  "gene_symbol": "GTF2IRD2"
}